optic nerve development [GO:0021554] (biological process) Also known as: cranial nerve 2 development, cranial nerve II development, CN II development Sources: GOC:cls, GOC:dgh, GOC:dph, GOC:jid, GO_REF:0000021 Definition: The process whose specific outcome is the progression of the optic nerve over time, from its formation to the mature structure. The sensory optic nerve originates from the bipolar cells of the retina and conducts visual information to the brainstem. The optic nerve exits the back of the eye in the orbit, enters the optic canal, and enters the central nervous system at the optic chiasm (crossing) where the nerve fibers become the optic tract just prior to entering the hindbrain. Relationships: is a type of GO:0021545